phosphoglycerate dehydrogenase activity [GO:0004617] (molecular function) Sources: EC:1.1.1.95 Definition: Catalysis of the reaction: 3-phosphoglycerate + NAD+ = 3-phosphohydroxypyruvate + NADH + H+. Relationships: is a type of oxidoreductase activity, acting on the CH-OH group of donors, NAD or NADP as acceptor [GO:0016616] Also known as: 3-phospho-D-glycerate:NAD+ 2-oxidoreductase activity, 3-phosphoglycerate dehydrogenase activity, 3-phosphoglycerate:NAD+ 2-oxidoreductase activity, 3-phosphoglyceric acid dehydrogenase activity, 3PHP reductase activity, D- and L-HGA, D-3-phosphoglycerate dehydrogenase activity, D-3-phosphoglycerate:NAD+ oxidoreductase activity, PGDH activity, SerA, SerA 3PG dehydrogenase activity, alpha-KG reductase activity, alpha-phosphoglycerate dehydrogenase activity, alphaKG reductase activity, glycerate 3-phosphate dehydrogenase activity, glycerate-1,3-phosphate dehydrogenase activity, phosphoglycerate oxidoreductase activity, phosphoglyceric acid dehydrogenase activity